{
  "gene_name": "Sperm acrosome membrane-associated protein 1",
  "gene": "UniProtKB:Q9HBV2",
  "term_label": "Unknown molecular function",
  "gene_symbol": "SPACA1",
  "term_id": "UNKNOWN:0001"
}